{
  "term_label": "homophilic cell-cell adhesion",
  "term_id": "GO:0007156",
  "gene_symbol": "MYOT",
  "gene": "UniProtKB:Q9UBF9",
  "gene_name": "Myotilin"
}